red or far-red light signaling pathway [GO:0010017] (biological process) Regulation: regulated by regulation of red or far-red light signaling pathway [GO:0090227]; positively regulated by GO:0090228; negatively regulated by GO:0090229 Sources: GOC:lr, GOC:mtg_far_red, GOC:sm Definition: The series of molecular signals initiated upon sensing by photoreceptor molecules of red light or far red light. Red light is electromagnetic radiation of wavelength of 580-700nm. Far red light is electromagnetic radiation of wavelength 700-800nm. An example of this response is seen at the beginning of many plant species developmental stages. These include germination, and the point when cotyledon expansion is triggered. In certain species these processes take place in response to absorption of red light by the pigment molecule phytochrome, but the signal can be reversed by exposure to far red light. During the initial phase the phytochrome molecule is only present in the red light absorbing form, but on absorption of red light it changes to a far red light absorbing form, triggering progress through development. An immediate short period of exposure to far red light entirely returns the pigment to its initial state and prevents triggering of the developmental process. A thirty minute break between red and subsequent far red light exposure renders the red light effect irreversible, and development then occurs regardless of whether far red light exposure subsequently occurs. Relationships: is a type of GO:0007165; is a type of cellular response to red or far red light [GO:0071489] Subtypes: far-red light signaling pathway [GO:0010018], GO:0010161 Also known as: phytochrome signaling pathway, red or far red light signaling pathway, red or far-red light signal transduction, red or far-red light signalling pathway, red/far red light signaling pathway